monoterpenol beta-glucosyltransferase activity [GO:0047219] (molecular function) Also known as: UDP-glucose:(-)-menthol O-beta-D-glucosyltransferase activity, UDPglucose:(-)-menthol O-beta-D-glucosyltransferase activity, UDPglucose:monoterpenol glucosyltransferase activity, uridine diphosphoglucose-monoterpenol glucosyltransferase activity Sources: EC:2.4.1.127, RHEA:11520 Relationships: is a type of UDP-glucosyltransferase activity [GO:0035251] Definition: Catalysis of the reaction: (-)-menthol + UDP-D-glucose = (-)-menthyl beta-D-glucoside + H+ + UDP.